negative regulation of renal sodium excretion by angiotensin [GO:0035820] (biological process) Sources: GOC:mtg_25march11, GOC:yaf Definition: The process in which angiotensin decreases the amount of sodium that is excreted in urine over a unit of time. Relationships: is a type of negative regulation of renal output by angiotensin [GO:0003083]; is a type of negative regulation of renal sodium excretion [GO:0035814]